cortical rotation [GO:0160174] (biological process) Definition: A cellular developmental process by which the outer layer of the cell (the cortex) rotates relative to the inner cytoplasm. References: PMID:22949618, PMID:25077289, PMID:37983969 Relationships: is_a cellular developmental process [GO:0048869]